cellular response to sucrose stimulus [GO:0071329] (biological process) Relationships: is a type of response to sucrose [GO:0009744]; is a type of cellular response to disaccharide stimulus [GO:0071324] Sources: GOC:mah Definition: Any process that results in a change in state or activity of a cell (in terms of movement, secretion, enzyme production, gene expression, etc.) as a result of a sucrose stimulus.